costamere [GO:0043034] (CC) Relationships: is a type of cellular anatomical structure [GO:0110165]; is part of myofibril [GO:0030016] References: PMID:6405378 Sources: GOC:jl, GOC:mtg_muscle, ISBN:0198506732 Definition: Regular periodic sub membranous arrays of vinculin in skeletal and cardiac muscle cells, these arrays link Z-discs to the sarcolemma and are associated with links to extracellular matrix.